periphagosomal region of cytoplasm [GO:1990783] (cellular component) References: PMID:18250451 Definition: Cytoplasm situated near, or occurring around, a phagosome. Relationships: is a type of cellular anatomical structure [GO:0110165]; is part of cytoplasm [GO:0005737]